{
  "gene_name": "Acyl-coenzyme A oxidase-like protein",
  "gene": "UniProtKB:Q9NUZ1",
  "term_id": "GO:0003997",
  "gene_symbol": "ACOXL",
  "term_label": "acyl-CoA oxidase activity"
}